{
  "term_label": "olfactory receptor activity",
  "term_id": "GO:0004984",
  "gene_symbol": "OR52I2",
  "gene_name": "Olfactory receptor 52I2",
  "gene": "UniProtKB:Q8NH67"
}